dermatome development [GO:0061054] (BP) Definition: The progression of the dermatome over time, from its initial formation to the mature structure. The dermatome is the portion of a somite that will form skin. Relationships: is a type of anatomical structure development [GO:0048856]; is part of GO:0061053 Sources: GOC:dph Regulation: regulated by regulation of dermatome development [GO:0061183]; positively regulated by positive regulation of dermatome development [GO:0061184]; negatively regulated by GO:0061185